{
  "term_label": "guanyl-nucleotide exchange factor activity",
  "gene_symbol": "MCF2L2",
  "gene": "UniProtKB:Q86YR7",
  "term_id": "GO:0005085",
  "gene_name": "Probable guanine nucleotide exchange factor MCF2L2"
}